negative regulation of fatty acid beta-oxidation using acyl-CoA dehydrogenase [GO:1904736] (biological process) Definition: Any process that stops, prevents or reduces the frequency, rate or extent of fatty acid beta-oxidation using acyl-CoA dehydrogenase. References: PMID:25416781 Sources: GOC:TermGenie, GO_REF:0000058 Also known as: down regulation of fatty acid beta-oxidation using acyl-CoA dehydrogenase, down-regulation of fatty acid beta-oxidation using acyl-CoA dehydrogenase, downregulation of fatty acid beta-oxidation using acyl-CoA dehydrogenase, inhibition of fatty acid beta-oxidation using acyl-CoA dehydrogenase Relationships: is_a GO:0031999; is_a regulation of fatty acid beta-oxidation using acyl-CoA dehydrogenase [GO:1904735]; negatively regulates fatty acid beta-oxidation using acyl-CoA dehydrogenase [GO:0033539]